{
  "term_id": "GO:0019731",
  "gene_symbol": "IGHD",
  "gene": "UniProtKB:P01880",
  "gene_name": "Immunoglobulin heavy constant delta",
  "term_label": "antibacterial humoral response"
}